{
  "gene": "UniProtKB:Q14699",
  "gene_symbol": "RFTN1",
  "gene_name": "Raftlin",
  "term_id": "UNKNOWN:0002",
  "term_label": "Unknown biological process"
}